{
  "gene": "UniProtKB:Q9UBK5",
  "term_id": "GO:0043548",
  "term_label": "phosphatidylinositol 3-kinase binding",
  "gene_symbol": "HCST",
  "gene_name": "Hematopoietic cell signal transducer"
}